positive regulation of progesterone secretion [GO:2000872] (biological process) Definition: Any process that activates or increases the frequency, rate or extent of progesterone secretion. Sources: GOC:sl Relationships: is a type of positive regulation of female gonad development [GO:2000196]; is a type of GO:2000833; is a type of regulation of progesterone secretion [GO:2000870]; positively regulates progesterone secretion [GO:0042701]